{
  "gene_symbol": "KCNA2",
  "term_label": "voltage-gated potassium channel complex",
  "gene_name": "Potassium voltage-gated channel subfamily A member 2",
  "term_id": "GO:0008076",
  "gene": "UniProtKB:P16389"
}